{
  "gene_name": "Cytochrome b-c1 complex subunit 7",
  "term_id": "GO:0006122",
  "gene": "UniProtKB:P14927",
  "term_label": "mitochondrial electron transport, ubiquinol to cytochrome c",
  "gene_symbol": "UQCRB"
}